{
  "gene_name": "STARD3 N-terminal-like protein",
  "term_id": "GO:0099044",
  "gene_symbol": "STARD3NL",
  "gene": "UniProtKB:O95772",
  "term_label": "vesicle tethering to endoplasmic reticulum"
}